{
  "gene": "UniProtKB:P0C7H9",
  "gene_symbol": "USP17L7",
  "gene_name": "Inactive ubiquitin carboxyl-terminal hydrolase 17-like protein 7",
  "term_id": "GO:0031647",
  "term_label": "regulation of protein stability"
}